benzoylformate decarboxylase activity [GO:0050695] (molecular function) Definition: Catalysis of the reaction: benzoylformate = benzaldehyde + CO2. Also known as: phenylglyoxylate decarboxylase activity, benzoylformate carboxy-lyase (benzaldehyde-forming), benzoylformate carboxy-lyase activity Sources: EC:4.1.1.7, MetaCyc:BENZOYLFORMATE-DECARBOXYLASE-RXN Relationships: is a type of carboxy-lyase activity [GO:0016831]